{
  "gene": "UniProtKB:Q9ULZ1",
  "gene_name": "Apelin",
  "term_id": "UNKNOWN:0002",
  "term_label": "Unknown biological process",
  "gene_symbol": "APLN"
}